{
  "term_id": "GO:0000981",
  "term_label": "DNA-binding transcription factor activity, RNA polymerase II-specific",
  "gene_name": "Signal transducer and activator of transcription 2",
  "gene": "UniProtKB:P52630",
  "gene_symbol": "STAT2"
}